actin cytoskeleton [GO:0015629] (cellular component) Definition: The part of the cytoskeleton (the internal framework of a cell) composed of actin and associated proteins. Includes actin cytoskeleton-associated complexes. Sources: GOC:jl, ISBN:0395825172, ISBN:0815316194 Relationships: is a type of cytoskeleton [GO:0005856] Subtypes: postsynaptic actin cytoskeleton [GO:0098871], presynaptic actin cytoskeleton [GO:0099143]